regulation of proline import across plasma membrane [GO:1902834] (biological process) Relationships: is a type of regulation of amino acid import across plasma membrane [GO:0010958]; is a type of regulation of organic acid transport [GO:0032890]; RO_0002211 proline import across plasma membrane [GO:1905647] Definition: Any process that modulates the frequency, rate or extent of proline import into cell. Also known as: regulation of proline import into cell Subtypes: negative regulation of proline import across plasma membrane [GO:1902835], GO:1902836, regulation of L-proline import across plasma membrane [GO:1905735] References: PMID:24344203 Sources: GOC:TermGenie, GO_REF:0000058